positive regulation of intrinsic apoptotic signaling pathway in response to DNA damage by p53 class mediator [GO:1902167] (biological process) Also known as: up regulation of intrinsic apoptotic signaling pathway in response to DNA damage by p53 class mediator, up-regulation of intrinsic apoptotic signaling pathway in response to DNA damage by p53 class mediator, upregulation of intrinsic apoptotic signaling pathway in response to DNA damage by p53 class mediator, activation of intrinsic apoptotic signaling pathway in response to DNA damage by p53 class mediator, activation of DNA damage response, signal transduction by p53 class mediator resulting in induction of apoptosis, positive regulation of DNA damage response, signal transduction by p53 class mediator resulting in induction of apoptosis, up regulation of DNA damage response, signal transduction by p53 class mediator resulting in induction of apoptosis, up-regulation of DNA damage response, signal transduction by p53 class mediator resulting in induction of apoptosis, upregulation of DNA damage response, signal transduction by p53 class mediator resulting in induction of apoptosis References: PMID:17719541 Sources: GOC:TermGenie Relationships: is a type of regulation of intrinsic apoptotic signaling pathway in response to DNA damage by p53 class mediator [GO:1902165]; is a type of positive regulation of intrinsic apoptotic signaling pathway in response to DNA damage [GO:1902231]; is a type of positive regulation of intrinsic apoptotic signaling pathway by p53 class mediator [GO:1902255]; positively regulates intrinsic apoptotic signaling pathway in response to DNA damage by p53 class mediator [GO:0042771] Definition: Any process that activates or increases the frequency, rate or extent of intrinsic apoptotic signaling pathway in response to DNA damage by p53 class mediator.